{
  "gene": "UniProtKB:Q9P2S2",
  "term_label": "trans-synaptic protein complex",
  "term_id": "GO:0098820",
  "gene_symbol": "NRXN2",
  "gene_name": "Neurexin-2"
}